{
  "gene": "UniProtKB:Q13503",
  "term_label": "transcription coregulator activity",
  "term_id": "GO:0003712",
  "gene_symbol": "MED21",
  "gene_name": "Mediator of RNA polymerase II transcription subunit 21"
}